{
  "term_label": "cytoplasm",
  "term_id": "GO:0005737",
  "gene_name": "Putative tripartite motif-containing protein 49B",
  "gene": "UniProtKB:A6NDI0",
  "gene_symbol": "TRIM49B"
}